{
  "term_label": "Unknown biological process",
  "gene_symbol": "LCE1F",
  "gene_name": "Late cornified envelope protein 1F",
  "gene": "UniProtKB:Q5T754",
  "term_id": "UNKNOWN:0002"
}